{
  "gene": "UniProtKB:P52907",
  "gene_name": "F-actin-capping protein subunit alpha-1",
  "term_id": "GO:0051016",
  "gene_symbol": "CAPZA1",
  "term_label": "barbed-end actin filament capping"
}